{
  "gene_name": "Caspase recruitment domain-containing protein 18",
  "gene": "UniProtKB:P57730",
  "term_label": "Unknown cellular component",
  "term_id": "UNKNOWN:0003",
  "gene_symbol": "CARD18"
}